interleukin-20 production [GO:0032624] (biological process) Regulation: regulated by regulation of interleukin-20 production [GO:0032664]; negatively regulated by negative regulation of interleukin-20 production [GO:0032704]; RO_0002213 by GO:0032744 Sources: GOC:mah Relationships: is a type of cytokine production [GO:0001816] Also known as: IL-20 production, ZCYTO10 production, interleukin-20 biosynthetic process, interleukin-20 secretion Definition: The appearance of interleukin-20 due to biosynthesis or secretion following a cellular stimulus, resulting in an increase in its intracellular or extracellular levels.